{
  "gene_name": "Kinesin-like protein KIF1A",
  "gene": "UniProtKB:Q12756",
  "term_id": "GO:0005737",
  "gene_symbol": "KIF1A",
  "term_label": "cytoplasm"
}